ciliary neurotrophic factor receptor binding [GO:0005127] (molecular function) Sources: GOC:ai Relationships: is_a cytokine receptor binding [GO:0005126] Definition: Binding to a ciliary neurotrophic factor receptor. Also known as: ciliary neurotrophic factor, ciliary neurotrophic factor receptor ligand